antigen processing and presentation of exogenous protein antigen via MHC class Ib, TAP-independent [GO:0002482] (biological process) References: PMID:15928678 Sources: GOC:add Also known as: TAP-independent antigen processing and presentation of exogenous peptide antigen via MHC class Ib, TAP-independent exogenous peptide antigen processing and presentation via MHC class Ib, exogenous peptide antigen processing and presentation via MHC class Ib, TAP-independent Relationships: is a type of GO:0002477 Definition: The process in which an antigen-presenting cell expresses a peptide antigen of exogenous origin on its cell surface in association with an MHC class Ib protein complex following intracellular transport via a pathway not requiring TAP (transporter associated with antigen processing). The peptide is typically a fragment of a larger exogenous protein which has been degraded within the cell. Class Ib here refers to non-classical class I molecules, such as those of the HLA-E gene family.